{
  "gene_symbol": "FABP2",
  "gene_name": "Fatty acid-binding protein, intestinal",
  "term_label": "cytosol",
  "term_id": "GO:0005829",
  "gene": "UniProtKB:P12104"
}